meiotic metaphase II chromosome alignment [GO:0043061] (biological process) References: PMID:10809666 Definition: A chromosome localization process whereby chromosomes are positioned in a specific order and orientation at the metaphase plate (spindle equator), during meiosis II chromosome segregation. This alignment ensures that each daughter cell will receive the correct number of chromosomes during cell division. Relationships: is a type of GO:0051311; is part of meiotic sister chromatid segregation [GO:0045144]